{
  "term_id": "GO:0019774",
  "gene_name": "Proteasome subunit beta type-6",
  "gene": "UniProtKB:P28072",
  "gene_symbol": "PSMB6",
  "term_label": "proteasome core complex, beta-subunit complex"
}